positive regulation of ARF protein signal transduction [GO:0032014] (biological process) Relationships: is a type of regulation of ARF protein signal transduction [GO:0032012]; is a type of positive regulation of small GTPase mediated signal transduction [GO:0051057]; positively regulates ARF protein signal transduction [GO:0032011] Sources: GOC:mah Definition: Any process that activates or increases the frequency, rate or extent of ARF protein signal transduction. Also known as: up regulation of ARF protein signal transduction, up-regulation of ARF protein signal transduction, upregulation of ARF protein signal transduction, activation of ARF protein signal transduction, stimulation of ARF protein signal transduction